neutrophil differentiation [GO:0030223] (biological process) Relationships: is a type of granulocyte differentiation [GO:0030851] Also known as: neutrophil cell differentiation, neutrophil granulocyte differentiation, neutrophil granulocytopoiesis Definition: The process in which a myeloid precursor cell acquires the specialized features of a neutrophil. Regulation: regulated by regulation of neutrophil differentiation [GO:0045658]; negatively regulated by negative regulation of neutrophil differentiation [GO:0045659]; positively regulated by positive regulation of neutrophil differentiation [GO:0045660] Sources: GOC:mah